{
  "gene_symbol": "SLC5A3",
  "gene": "UniProtKB:P53794",
  "gene_name": "Sodium_myo-inositol cotransporter",
  "term_label": "Unknown biological process",
  "term_id": "UNKNOWN:0002"
}